{
  "gene_name": "C-C motif chemokine 19",
  "term_label": "extracellular space",
  "gene_symbol": "CCL19",
  "term_id": "GO:0005615",
  "gene": "UniProtKB:Q99731"
}